interleukin-17 binding [GO:0019975] (molecular function) Subtypes: interleukin-25 binding [GO:0045511], interleukin-27 binding [GO:0045513] Definition: Binding to a member of the interleukin-17 family of cytokines. Also known as: IL-17 binding Sources: GOC:add, GOC:jl Relationships: is a type of cytokine binding [GO:0019955]